positive regulation of meiosis I [GO:0060903] (biological process) Sources: GOC:dph, GOC:tb Relationships: is a type of positive regulation of meiotic nuclear division [GO:0045836]; is a type of regulation of meiosis I [GO:0060631]; positively regulates GO:0007127 Definition: Any process that increases the rate, frequency, or extent of meiosis I, a cell cycle process comprising the steps by which a cell progresses through the first phase of meiosis, in which cells divide and homologous chromosomes are paired and segregated from each other, producing two daughter cells.